{
  "gene_name": "Testis-expressed protein 15",
  "gene": "UniProtKB:Q9BXT5",
  "term_label": "synaptonemal complex assembly",
  "gene_symbol": "TEX15",
  "term_id": "GO:0007130"
}